{
  "term_label": "plasma membrane",
  "gene": "UniProtKB:Q15303",
  "gene_name": "Receptor tyrosine-protein kinase erbB-4",
  "gene_symbol": "ERBB4",
  "term_id": "GO:0005886"
}